{
  "gene_name": "Rho guanine nucleotide exchange factor 1",
  "gene": "UniProtKB:Q92888",
  "term_label": "G protein-coupled receptor binding",
  "gene_symbol": "ARHGEF1",
  "term_id": "GO:0001664"
}